{
  "gene": "UniProtKB:A6NJV1",
  "gene_name": "Protein FAM166C",
  "term_label": "Unknown molecular function",
  "gene_symbol": "FAM166C",
  "term_id": "UNKNOWN:0001"
}